{
  "gene_symbol": "LHX8",
  "term_id": "GO:0005634",
  "gene_name": "LIM_homeobox protein Lhx8",
  "term_label": "nucleus",
  "gene": "UniProtKB:Q68G74"
}